embryonic heart tube morphogenesis [GO:0003143] (biological process) Subtypes: GO:0001947, heart jogging [GO:0003146] Sources: GOC:mtg_heart Definition: The process in which the anatomical structures of the embryonic heart tube are generated and organized. The embryonic heart tube is an epithelial tube that will give rise to the mature heart. Relationships: is a type of embryonic morphogenesis [GO:0048598]; is_a epithelial tube morphogenesis [GO:0060562]; is part of GO:0003007; is part of embryonic heart tube development [GO:0035050]; BFO_0000050 embryonic organ morphogenesis [GO:0048562]